{
  "term_id": "UNKNOWN:0003",
  "term_label": "Unknown cellular component",
  "gene": "UniProtKB:Q8N7X1",
  "gene_name": "RNA-binding motif protein, X-linked-like-3",
  "gene_symbol": "RBMXL3"
}